{
  "term_id": "GO:0030424",
  "gene_name": "Rap1 GTPase-activating protein 1",
  "gene": "UniProtKB:P47736",
  "term_label": "axon",
  "gene_symbol": "RAP1GAP"
}